{
  "gene_name": "Gap junction beta-3 protein",
  "term_id": "GO:0007267",
  "gene": "UniProtKB:O75712",
  "gene_symbol": "GJB3",
  "term_label": "cell-cell signaling"
}